AP-2 adaptor complex [GO:0030122] (CC) References: PMID:10611976, PMID:21097499, PMID:22022230, PMID:24322426 Sources: GOC:mah Also known as: HA2, HA2 clathrin adaptor Relationships: is a type of clathrin adaptor complex [GO:0030131]; is a type of plasma membrane protein complex [GO:0098797]; is part of clathrin coat of endocytic vesicle [GO:0030128]; is part of clathrin coat of coated pit [GO:0030132] Definition: A heterotetrameric AP-type membrane coat adaptor complex that consists of alpha, beta2, mu2 and sigma2 subunits, and links clathrin to the membrane surface of a vesicle, and the cargo receptors during receptor/clathrin mediated endocytosis. Vesicles with AP-2-containing coats are normally found primarily near the plasma membrane, on endocytic vesicles. In at least humans, the AP-2 complex can be heterogeneric due to the existence of multiple subunit isoforms encoded by different alpha genes (alphaA and alphaC).